{
  "term_label": "phosphatidylinositol-3,4,5-trisphosphate binding",
  "gene_symbol": "ARAP2",
  "gene_name": "Arf-GAP with Rho-GAP domain, ANK repeat and PH domain-containing protein 2",
  "gene": "UniProtKB:Q8WZ64",
  "term_id": "GO:0005547"
}